{
  "term_id": "GO:0005634",
  "gene_name": "Protein LYRIC",
  "term_label": "nucleus",
  "gene_symbol": "MTDH",
  "gene": "UniProtKB:Q86UE4"
}